TAP complex [GO:0042825] (cellular component) Relationships: is a type of membrane protein complex [GO:0098796]; is a type of endoplasmic reticulum protein-containing complex [GO:0140534]; is part of MHC class I peptide loading complex [GO:0042824] References: PMID:10618487, PMID:10631934 Sources: GOC:jl Also known as: transporter associated with antigen presentation Definition: A heterodimer composed of the subunits TAP1 and TAP2 (transporter associated with antigen presentation). Functions in the transport of antigenic peptides from the cytosol to the lumen of the endoplasmic reticulum.